{
  "gene": "UniProtKB:Q6UXV0",
  "term_id": "GO:0038023",
  "gene_symbol": "GFRAL",
  "term_label": "signaling receptor activity",
  "gene_name": "GDNF family receptor alpha-like"
}